{
  "gene_symbol": "PAX9",
  "gene": "UniProtKB:P55771",
  "gene_name": "Paired box protein Pax-9",
  "term_id": "GO:0000978",
  "term_label": "RNA polymerase II cis-regulatory region sequence-specific DNA binding"
}